{
  "term_id": "GO:0008266",
  "term_label": "poly(U) RNA binding",
  "gene_symbol": "RBMS2",
  "gene": "UniProtKB:Q15434",
  "gene_name": "RNA-binding motif, single-stranded-interacting protein 2"
}